{
  "gene": "UniProtKB:P12034",
  "gene_name": "Fibroblast growth factor 5",
  "term_label": "fibroblast growth factor receptor signaling pathway",
  "gene_symbol": "FGF5",
  "term_id": "GO:0008543"
}